positive regulation of anterior/posterior axon guidance [GO:1905488] (biological process) Relationships: is a type of positive regulation of axon guidance [GO:1902669]; is a type of regulation of anterior/posterior axon guidance [GO:1905486]; positively regulates anterior/posterior axon guidance [GO:0033564] Definition: Any process that activates or increases the frequency, rate or extent of anterior/posterior axon guidance. References: PMID:16516839 Sources: GOC:TermGenie, GO_REF:0000058 Also known as: positive regulation of anterior-posterior axon guidance, positive regulation of anterior/posterior axon pathfinding, up regulation of anterior-posterior axon guidance, up regulation of anterior/posterior axon guidance, up regulation of anterior/posterior axon pathfinding, up-regulation of anterior-posterior axon guidance, up-regulation of anterior/posterior axon guidance, up-regulation of anterior/posterior axon pathfinding, upregulation of anterior-posterior axon guidance, upregulation of anterior/posterior axon guidance, upregulation of anterior/posterior axon pathfinding, activation of anterior-posterior axon guidance, activation of anterior/posterior axon guidance, activation of anterior/posterior axon pathfinding